2-hydroxyphytanoyl-CoA lyase activity [GO:0106376] (molecular function) Definition: Catalysis of the reaction: 2-hydroxyphytanoyl-CoA = 2,6,10,14-tetramethylpentadecanal + formyl-CoA. Relationships: is a type of 2-hydroxyacyl-CoA lyase activity [GO:0106359] References: PMID:10468558 Sources: RHEA:25355